{
  "gene_name": "DNA polymerase epsilon catalytic subunit A",
  "term_label": "single-stranded DNA 3'-5' DNA exonuclease activity",
  "gene_symbol": "POLE",
  "gene": "UniProtKB:Q07864",
  "term_id": "GO:0008310"
}